{
  "term_label": "mitochondrion",
  "term_id": "GO:0005739",
  "gene_name": "ATPase family AAA domain-containing protein 3B",
  "gene_symbol": "ATAD3B",
  "gene": "UniProtKB:Q5T9A4"
}